{
  "term_id": "GO:0000785",
  "gene": "UniProtKB:O43482",
  "gene_name": "Protein Mis18-beta",
  "term_label": "chromatin",
  "gene_symbol": "OIP5"
}